pupation [GO:0035074] (biological process) Relationships: is a type of GO:0032501; is part of pupal development [GO:0035209] Sources: GOC:bf, ISBN:0582227089, ISBN:0879694238 Definition: The act of becoming a pupa, a resting stage in the life cycle of organisms with complete metamorphosis. This event marks the end of the prepupal period and the beginning of the pupal period. Also known as: head eversion, prepupal-pupal transition